{
  "gene_name": "Calcium uptake protein 3, mitochondrial",
  "gene": "UniProtKB:Q86XE3",
  "gene_symbol": "MICU3",
  "term_id": "GO:0051560",
  "term_label": "mitochondrial calcium ion homeostasis"
}